{
  "term_label": "cytoplasm",
  "gene": "UniProtKB:Q15020",
  "term_id": "GO:0005737",
  "gene_symbol": "SART3",
  "gene_name": "Squamous cell carcinoma antigen recognized by T-cells 3"
}